{
  "term_id": "GO:0042593",
  "term_label": "glucose homeostasis",
  "gene_name": "Fibrillin-1",
  "gene_symbol": "FBN1",
  "gene": "UniProtKB:P35555"
}